{
  "gene_symbol": "RAD9A",
  "term_id": "GO:0030896",
  "term_label": "checkpoint clamp complex",
  "gene_name": "Cell cycle checkpoint control protein RAD9A",
  "gene": "UniProtKB:Q99638"
}